{
  "term_label": "Unknown molecular function",
  "gene_name": "Testis-expressed protein 35",
  "term_id": "UNKNOWN:0001",
  "gene_symbol": "TEX35",
  "gene": "UniProtKB:Q5T0J7"
}